{
  "gene_symbol": "A8MU10",
  "term_id": "UNKNOWN:0002",
  "gene": "UniProtKB:A8MU10",
  "term_label": "Unknown biological process",
  "gene_name": "Putative uncharacterized protein ENSP00000381562"
}